endoplasmic reticulum to chloroplast transport [GO:1901965] (biological process) Also known as: ER to chloroplast transport References: PMID:18689504 Sources: GOC:TermGenie Relationships: is a type of intracellular transport [GO:0046907] Definition: The directed movement of substances from endoplasmic reticulum to chloroplast. Subtypes: GO:1990052